{
  "gene_symbol": "OR5M9",
  "term_id": "GO:0007608",
  "gene_name": "Olfactory receptor 5M9",
  "term_label": "sensory perception of smell",
  "gene": "UniProtKB:Q8NGP3"
}